{
  "gene_symbol": "GRK1",
  "gene": "UniProtKB:Q15835",
  "gene_name": "Rhodopsin kinase GRK1",
  "term_label": "cytoplasm",
  "term_id": "GO:0005737"
}